{
  "gene_name": "POU class 2 homeobox associating factor 3",
  "gene_symbol": "POU2AF3",
  "term_id": "UNKNOWN:0002",
  "gene": "UniProtKB:A8K830",
  "term_label": "Unknown biological process"
}